ocellus photoreceptor cell fate commitment [GO:0042707] (BP) Definition: The process in which the developmental fate of a cell becomes restricted such that it will develop into photoreceptor cell in the ocellus. A photoreceptor cell is a cell that responds to incident electromagnetic radiation. Different classes of photoreceptor have different spectral sensitivities and express different photosensitive pigments. Sources: GOC:mtg_sensu Relationships: is a type of photoreceptor cell fate commitment [GO:0046552]; is part of GO:0042705